{
  "gene": "UniProtKB:Q9UNY5",
  "gene_symbol": "ZNF232",
  "gene_name": "Zinc finger protein 232",
  "term_label": "RNA polymerase II cis-regulatory region sequence-specific DNA binding",
  "term_id": "GO:0000978"
}